{
  "term_id": "GO:0007210",
  "gene": "UniProtKB:P41595",
  "gene_name": "5-hydroxytryptamine receptor 2B",
  "term_label": "serotonin receptor signaling pathway",
  "gene_symbol": "HTR2B"
}